{
  "term_label": "ERAD pathway",
  "gene_symbol": "TMUB2",
  "term_id": "GO:0036503",
  "gene_name": "Transmembrane and ubiquitin-like domain-containing protein 2",
  "gene": "UniProtKB:Q71RG4"
}